glycyrrhetinate biosynthetic process [GO:1902386] (biological process) References: PMID:22128119 Sources: GOC:TermGenie Also known as: glycyrrhetinate anabolism, glycyrrhetinate biosynthesis, glycyrrhetinate formation, glycyrrhetinate synthesis Definition: The chemical reactions and pathways resulting in the formation of glycyrrhetinate. Relationships: is a type of pentacyclic triterpenoid biosynthetic process [GO:0019745]; is a type of ketone biosynthetic process [GO:0042181]; is a type of GO:0072330